{
  "gene": "UniProtKB:A1L190",
  "gene_symbol": "SYCE3",
  "term_id": "GO:0007131",
  "gene_name": "Synaptonemal complex central element protein 3",
  "term_label": "reciprocal meiotic recombination"
}